positive regulation of mesenchymal stem cell proliferation [GO:1902462] (biological process) Relationships: is_a regulation of mesenchymal stem cell proliferation [GO:1902460]; is a type of positive regulation of stem cell proliferation [GO:2000648]; positively regulates mesenchymal stem cell proliferation [GO:0097168] Also known as: positive regulation of MSC proliferation, up regulation of MSC proliferation, up regulation of mesenchymal stem cell proliferation, up-regulation of MSC proliferation, up-regulation of mesenchymal stem cell proliferation, upregulation of MSC proliferation, upregulation of mesenchymal stem cell proliferation, activation of MSC proliferation, activation of mesenchymal stem cell proliferation References: PMID:18672106 Sources: GOC:TermGenie, GOC:pm Definition: Any process that activates or increases the frequency, rate or extent of mesenchymal stem cell proliferation.